{
  "term_id": "GO:0035098",
  "gene": "UniProtKB:O75530",
  "gene_symbol": "EED",
  "gene_name": "Polycomb protein EED",
  "term_label": "ESC/E(Z) complex"
}